{
  "term_id": "GO:0005634",
  "gene_symbol": "ZNF689",
  "gene": "UniProtKB:Q96CS4",
  "term_label": "nucleus",
  "gene_name": "Zinc finger protein 689"
}